positive regulation of vascular associated smooth muscle cell dedifferentiation [GO:1905176] (biological process) References: PMID:19088079 Sources: GOC:BHF, GOC:BHF_miRNA, GOC:TermGenie, GOC:rph, GO_REF:0000058 Also known as: positive regulation of vascular smooth muscle cell dedifferentiation, up regulation of vascular smooth muscle cell dedifferentiation, up-regulation of vascular smooth muscle cell dedifferentiation, upregulation of vascular smooth muscle cell dedifferentiation, activation of vascular smooth muscle cell dedifferentiation Definition: Any process that activates or increases the frequency, rate or extent of vascular smooth muscle cell dedifferentiation. Relationships: is a type of GO:0048522; is a type of positive regulation of developmental process [GO:0051094]; is a type of regulation of vascular associated smooth muscle cell dedifferentiation [GO:1905174]; positively regulates vascular associated smooth muscle cell dedifferentiation [GO:1990936]